{
  "term_label": "cytoplasm",
  "term_id": "GO:0005737",
  "gene_name": "Phosducin-like protein 2",
  "gene_symbol": "PDCL2",
  "gene": "UniProtKB:Q8N4E4"
}